{
  "term_label": "Unknown cellular component",
  "term_id": "UNKNOWN:0003",
  "gene_name": "Uncharacterized protein CXorf38",
  "gene": "UniProtKB:Q8TB03",
  "gene_symbol": "CXorf38"
}